{
  "gene_name": "Calmodulin-2",
  "gene_symbol": "CALM2",
  "gene": "UniProtKB:P0DP24",
  "term_id": "GO:0005737",
  "term_label": "cytoplasm"
}